{
  "gene_symbol": "NPM1",
  "gene": "UniProtKB:P06748",
  "gene_name": "Nucleophosmin",
  "term_id": "GO:0005813",
  "term_label": "centrosome"
}